{
  "gene_symbol": "RBM25",
  "gene_name": "RNA-binding protein 25",
  "term_label": "mRNA binding",
  "term_id": "GO:0003729",
  "gene": "UniProtKB:P49756"
}